{
  "gene_symbol": "HMGXB3",
  "gene_name": "HMG domain-containing protein 3",
  "gene": "UniProtKB:Q12766",
  "term_label": "Unknown molecular function",
  "term_id": "UNKNOWN:0001"
}